{
  "gene_symbol": "VPS13C",
  "term_label": "protein retention in Golgi apparatus",
  "term_id": "GO:0045053",
  "gene": "UniProtKB:Q709C8",
  "gene_name": "Intermembrane lipid transfer protein VPS13C"
}